borate channel activity [GO:0180044] (molecular function) Definition: Enables the facilitated diffusion of borate (by an energy-independent process) involving passage through a transmembrane aqueous pore or channel without evidence for a carrier-mediated mechanism. References: PMID:21710975 Relationships: is a type of GO:0015267